{
  "term_label": "cholesterol transfer activity",
  "gene_symbol": "ABCG5",
  "gene_name": "ATP-binding cassette sub-family G member 5",
  "gene": "UniProtKB:Q9H222",
  "term_id": "GO:0120020"
}